{
  "term_label": "regulation of receptor internalization",
  "gene": "UniProtKB:O75955",
  "term_id": "GO:0002090",
  "gene_symbol": "FLOT1",
  "gene_name": "Flotillin-1"
}